{
  "gene": "UniProtKB:Q14154",
  "term_id": "GO:0043539",
  "term_label": "protein serine/threonine kinase activator activity",
  "gene_name": "DAP3-binding cell death enhancer 1",
  "gene_symbol": "DELE1"
}